{
  "gene_symbol": "ACSM6",
  "gene": "UniProtKB:Q6P461",
  "gene_name": "Acyl-coenzyme A synthetase ACSM6, mitochondrial",
  "term_id": "GO:0006637",
  "term_label": "acyl-CoA metabolic process"
}